dimethyl selenide methyltransferase activity [GO:0098615] (molecular function) Definition: Catalysis of the reaction: S-adenosyl-L-methionine + dimethyl selenide = S-adenosyl-L-homocysteine + trimethylselenonium. References: PMID:17988700, PMID:3350800 Relationships: is_a methyltransferase activity [GO:0008168]